taste receptor complex [GO:1903768] (cellular component) Relationships: is a type of receptor complex [GO:0043235] Definition: A protein complex which is capable of taste receptor activity. References: PMID:16720576 Sources: GOC:BHF, GOC:TermGenie, GOC:rl, GO_REF:0000088 Subtypes: GO:1903767